{
  "gene_name": "Adenylate kinase 8",
  "gene": "UniProtKB:Q96MA6",
  "term_label": "Unknown biological process",
  "gene_symbol": "AK8",
  "term_id": "UNKNOWN:0002"
}